presynaptic membrane assembly [GO:0097105] (biological process) Definition: The aggregation, arrangement and bonding together of a set of components to form a presynaptic membrane, including any proteins associated with the membrane, but excluding other cellular components. A presynaptic membrane is a specialized area of membrane of the axon terminal that faces the plasma membrane of the neuron or muscle fiber with which the axon terminal establishes a synaptic junction. References: PMID:15797875, PMID:18550748 Sources: GOC:BHF, GOC:pr, GOC:sjp Also known as: pre-synaptic membrane assembly Note: Note that 'presynaptic membrane' in this term should not be mistaken with 'presynaptic active zone'. The latter encompasses more than the former, as it also includes the specialized cortical cytoskeletal matrix in the cell cortex of a presynaptic neuron. Relationships: is a type of GO:0071709; is a type of presynaptic membrane organization [GO:0097090]; is part of GO:0099054